oxo-acid-lyase activity [GO:0016833] (molecular function) Relationships: is a type of carbon-carbon lyase activity [GO:0016830] Subtypes: anthranilate synthase activity [GO:0004049], GO:0004419, GO:0004451, GO:0008696, GO:0008700, 4-hydroxy-2-oxovalerate aldolase activity [GO:0008701], N-acetylneuraminate lyase activity [GO:0008747], GO:0008813, citrate (pro-3S)-lyase activity [GO:0008815], citryl-CoA lyase activity [GO:0008816], GO:0008935, L-erythro-3-methylmalyl-CoA lyase activity [GO:0043959], (3R)-citramalyl-CoA lyase activity [GO:0044101], methylisocitrate lyase activity [GO:0046421], GO:0047443, 3-hydroxy-3-isohexenylglutaryl-CoA lyase activity [GO:0047445], (1-hydroxycyclohexan-1-yl)acetyl-CoA lyase activity [GO:0047446], 2,3-dimethylmalate lyase activity [GO:0047529], 3-hydroxyaspartate aldolase activity [GO:0047562], citramalate lyase activity [GO:0047776], (S)-citramalyl-CoA lyase activity [GO:0047777], malyl-CoA lyase activity [GO:0050083], GO:0050204, GO:0102521, (4S)-4-hydroxy-2-oxoglutarate aldolase activity [GO:0106009] Sources: EC:4.1.3.-, GOC:jl Also known as: oxo-acid lyase activity, oxoacid lyase activity Definition: Catalysis of the cleavage of a C-C bond by other means than by hydrolysis or oxidation, of a 3-hydroxy acid.